stizolobinate synthase activity [GO:0050298] (molecular function) Also known as: 3,4-dihydroxy-L-phenylalanine:oxygen 2,3-oxidoreductase (recyclizing) Relationships: is a type of oxidoreductase activity, acting on single donors with incorporation of molecular oxygen, incorporation of two atoms of oxygen [GO:0016702] Sources: EC:1.13.11.30, MetaCyc:STIZOLOBINATE-SYNTHASE-RXN Definition: Catalysis of the reaction: 3,4-dihydroxy-L-phenylalanine + O2 = 5-(L-alanin-3-yl)-2-hydroxy-cis,cis-muconate 6-semialdehyde.